cerebellar Purkinje cell layer structural organization [GO:0021693] (biological process) Sources: GOC:cls, GOC:dgh, GOC:dph, GOC:jid, GO_REF:0000021 Relationships: is a type of anatomical structure arrangement [GO:0048532]; BFO_0000050 cerebellar Purkinje cell layer morphogenesis [GO:0021692]; is part of cerebellar cortex structural organization [GO:0021698] Also known as: cerebellar Purkinje cell layer structural organisation Definition: The process that contributes to the act of creating the structural organization of the cerebellar Purkinje cell layer. This process pertains to the physical shaping of a rudimentary structure. The Purkinje cell layer lies just underneath the molecular layer of the cerebellar cortex. It contains the neuronal cell bodies of the Purkinje cells that are arranged side by side in a single layer. Candelabrum interneurons are vertically oriented between the Purkinje cells. Purkinje neurons are inhibitory and provide the output of the cerebellar cortex through axons that project into the white matter. Extensive dendritic trees from the Purkinje cells extend upward in a single plane into the molecular layer where they synapse with parallel fibers of granule cells.